{
  "gene_symbol": "RIBC1",
  "gene": "UniProtKB:Q8N443",
  "term_id": "UNKNOWN:0001",
  "gene_name": "RIB43A-like with coiled-coils protein 1",
  "term_label": "Unknown molecular function"
}